{
  "gene_name": "Coiled-coil domain-containing protein 6",
  "gene_symbol": "CCDC6",
  "term_label": "Unknown cellular component",
  "term_id": "UNKNOWN:0003",
  "gene": "UniProtKB:Q16204"
}